{
  "gene": "UniProtKB:Q8IUC8",
  "gene_symbol": "GALNT13",
  "term_label": "Golgi apparatus",
  "gene_name": "Polypeptide N-acetylgalactosaminyltransferase 13",
  "term_id": "GO:0005794"
}